{
  "gene_symbol": "PPP1R12A",
  "gene": "UniProtKB:O14974",
  "term_id": "GO:0031672",
  "gene_name": "Protein phosphatase 1 regulatory subunit 12A",
  "term_label": "A band"
}